{
  "gene_name": "Lymphokine-activated killer T-cell-originated protein kinase",
  "term_id": "UNKNOWN:0002",
  "gene": "UniProtKB:Q96KB5",
  "term_label": "Unknown biological process",
  "gene_symbol": "PBK"
}